virion attachment to host cell flagellum [GO:0098931] (biological process) Definition: The process by which a virion attaches to a the host cell flagellum. Some DNA bacterial viruses use flagella to attach to the host cell. This contact with the flagellum facilitates concentration of phage particles around the entry receptor on the bacterial cell surface. Sources: GOC:dos, VZ:3949 Relationships: is_a virion attachment to host cell [GO:0019062]